microautophagy [GO:0016237] (biological process) Also known as: lysosomal microautophagy Subtypes: micromitophagy [GO:0000424], micropexophagy [GO:0000426], piecemeal microautophagy of the nucleus [GO:0034727], GO:0061738, microlipophagy [GO:0140504] Definition: A type of autophagy where cytosolic components are ingested by late endosomes, lysosomes or yeast-type lytic vacuoles by direct invagination of the compartment membrane without prior sequestration into an autophagosome. The engulfing membranes fuse, resulting in the lysosomal delivery of the cargo wrapped in a single membrane derived from the invaginated lysosomal membrane. Relationships: is a type of autophagy [GO:0006914] References: PMID:14679207, PMID:15798367, PMID:16973210, PMID:9566964